positive regulation of filamentous growth of a population of unicellular organisms in response to heat [GO:1900433] (biological process) Sources: GOC:TermGenie, GOC:di Relationships: is a type of GO:0048584; is a type of positive regulation of filamentous growth of a population of unicellular organisms [GO:1900430]; is a type of GO:1900431; positively regulates filamentous growth of a population of unicellular organisms in response to heat [GO:0036168] Definition: Any process that activates or increases the frequency, rate or extent of filamentous growth of a population of unicellular organisms in response to heat. Also known as: up regulation of filamentous growth of a population of unicellular organisms in response to heat, up-regulation of filamentous growth of a population of unicellular organisms in response to heat, upregulation of filamentous growth of a population of unicellular organisms in response to heat, activation of filamentous growth of a population of unicellular organisms in response to heat